{
  "gene_name": "Pituitary homeobox 1",
  "term_label": "regulation of transcription by RNA polymerase II",
  "gene_symbol": "PITX1",
  "gene": "UniProtKB:P78337",
  "term_id": "GO:0006357"
}